negative regulation of AIM2 inflammasome complex assembly [GO:0140972] (biological process) References: PMID:33467177 Relationships: is a type of GO:0031333; is a type of regulation of AIM2 inflammasome complex assembly [GO:0140971]; is part of GO:0141086; negatively regulates AIM2 inflammasome complex assembly [GO:0140970] Definition: Any process that stops, prevents or reduces the frequency, rate or extent of AIM2 inflammasome complex assembly.